{
  "gene": "UniProtKB:P48050",
  "term_label": "potassium ion import across plasma membrane",
  "gene_name": "Inward rectifier potassium channel 4",
  "gene_symbol": "KCNJ4",
  "term_id": "GO:1990573"
}